{
  "term_id": "UNKNOWN:0002",
  "gene": "UniProtKB:Q9Y2X3",
  "gene_symbol": "NOP58",
  "term_label": "Unknown biological process",
  "gene_name": "Nucleolar protein 58"
}